pentitol catabolic process [GO:0019527] (biological process) Sources: ISBN:0198506732 Relationships: is a type of alditol catabolic process [GO:0019405]; is a type of pentitol metabolic process [GO:0019519] Also known as: pentitol breakdown, pentitol catabolism, pentitol degradation Subtypes: ribitol catabolic process [GO:0046363], arabitol catabolic process [GO:0051157], xylitol catabolic process [GO:0051160] Definition: The chemical reactions and pathways resulting in the breakdown of pentitols, any alditol with a chain of five carbon atoms in the molecule.